N-acetyllactosaminide beta-1,3-N-acetylglucosaminyltransferase activity [GO:0008532] (molecular function) Definition: Catalysis of the reaction: a beta-D-galactosyl-(1->4)-N-acetyl-beta-D-glucosaminyl derivative + UDP-N-acetyl-alpha-D-glucosamine = an N-acetyl-beta-D-glucosaminyl-(1->3)-beta-D-galactosyl-(1->4)-N-acetyl-beta-D-glucosaminyl derivative + H+ + UDP. Sources: RHEA:14389 Also known as: poly-N-acetyllactosamine extension enzyme activity, uridine diphosphoacetylglucosamine-acetyllactosaminide beta-1,3-acetylglucosaminyltransferase, uridine diphosphoacetylglucosamine-acetyllactosaminide beta1->3-acetylglucosaminyltransferase, GnTE activity, N-acetyllactosamine beta(1,3)N-acetylglucosaminyltransferase activity, UDP-GlcNAc:GalR, beta-D-3-N-acetylglucosaminyltransferase activity, UDP-GlcNAc:Galbeta-(1,4)-GlcNAcbeta-r-beta-(1,3)-N-acetylglucosaminyltransferase activity, UDP-GlcNAc:Galbeta-1,4-GlcNAcbeta-beta-1,3-N-acetylglucosaminyltransferase activity, UDP-N-acetyl-D-glucosamine:beta-D-galactosyl-1,4-N-acetyl-D-glucosamine beta-1,3-acetyl-D-glucosaminyltransferase activity, galbeta1->4GlcNAc-R beta1->3 N-acetylglucosaminyltransferase activity Relationships: is a type of acetylglucosaminyltransferase activity [GO:0008375]